monoatomic ion transmembrane transporter activity [GO:0015075] (molecular function) Regulation: negatively regulated by negative regulation of ion transmembrane transporter activity [GO:0032413]; positively regulated by positive regulation of ion transmembrane transporter activity [GO:0032414] Definition: Enables the transfer of an ion from one side of a membrane to the other. Sources: GOC:dgf, GOC:mtg_transport, ISBN:0815340729 Subtypes: monoatomic ion channel activity [GO:0005216], monoatomic cation transmembrane transporter activity [GO:0008324], monoatomic anion transmembrane transporter activity [GO:0008509], active monoatomic ion transmembrane transporter activity [GO:0022853] Relationships: is a type of transmembrane transporter activity [GO:0022857]; is part of monoatomic ion transmembrane transport [GO:0034220] Also known as: ion transmembrane transporter activity, ion transporter activity